{
  "term_id": "GO:0031114",
  "gene": "UniProtKB:Q66K74",
  "term_label": "regulation of microtubule depolymerization",
  "gene_symbol": "MAP1S",
  "gene_name": "Microtubule-associated protein 1S"
}